{
  "term_id": "GO:0005886",
  "term_label": "plasma membrane",
  "gene_name": "Phospholipase D2",
  "gene": "UniProtKB:O14939",
  "gene_symbol": "PLD2"
}